{
  "gene_name": "Microtubule-associated protein 6",
  "gene_symbol": "MAP6",
  "term_id": "GO:0005801",
  "term_label": "cis-Golgi network",
  "gene": "UniProtKB:Q96JE9"
}